{
  "gene_name": "Ubiquitin carboxyl-terminal hydrolase 2",
  "term_id": "GO:0005737",
  "gene_symbol": "USP2",
  "gene": "UniProtKB:O75604",
  "term_label": "cytoplasm"
}